CA3 pyramidal cell dendrite [GO:0097442] (cellular component) Sources: NIF_Subcellular:nlx_subcell_1005001 Definition: A dendrite of a hippocampal CA3 pyramidal cell. Relationships: is a type of dendrite [GO:0030425]